{
  "gene_name": "Unconventional myosin-Va",
  "term_label": "actin filament organization",
  "term_id": "GO:0007015",
  "gene_symbol": "MYO5A",
  "gene": "UniProtKB:Q9Y4I1"
}